chromoplast intermembrane space [GO:0031973] (cellular component) Definition: The region between the inner and outer lipid bilayers of a chromoplast envelope. Also known as: chromoplast envelope lumen Relationships: is a type of plastid intermembrane space [GO:0009529]; BFO_0000050 chromoplast envelope [GO:0031898] Sources: GOC:mah